{
  "term_id": "GO:0001164",
  "gene": "UniProtKB:P17480",
  "gene_name": "Nucleolar transcription factor 1",
  "gene_symbol": "UBTF",
  "term_label": "RNA polymerase I core promoter sequence-specific DNA binding"
}